positive regulation of fibroblast growth factor receptor signaling pathway involved in ureteric bud formation [GO:2000704] (biological process) Sources: GOC:mtg_kidney_jan10, GOC:obol, GOC:yaf Definition: Any process that activates or increases the frequency, rate or extent of fibroblast growth factor receptor signaling pathway involved in ureteric bud formation. Also known as: positive regulation of FGF receptor signaling pathway of ureteric bud formation, positive regulation of FGF receptor signalling pathway of ureteric bud formation, positive regulation of FGFR signaling pathway of ureteric bud formation, positive regulation of fibroblast growth factor receptor signaling pathway of ureteric bud formation, positive regulation of fibroblast growth factor receptor signalling pathway of ureteric bud formation Relationships: is a type of positive regulation of fibroblast growth factor receptor signaling pathway [GO:0045743]; is a type of GO:2000702; positively regulates fibroblast growth factor receptor signaling pathway involved in ureteric bud formation [GO:2000699]